{
  "term_label": "regulation of gene expression",
  "gene_name": "Lysine-specific demethylase 4A",
  "gene": "UniProtKB:O75164",
  "term_id": "GO:0010468",
  "gene_symbol": "KDM4A"
}